{
  "term_label": "peroxisomal matrix",
  "gene_symbol": "DDO",
  "term_id": "GO:0005782",
  "gene_name": "D-aspartate oxidase",
  "gene": "UniProtKB:Q99489"
}